{
  "gene_symbol": "CYB561D2",
  "term_id": "GO:0005789",
  "gene": "UniProtKB:O14569",
  "gene_name": "Transmembrane reductase CYB561D2",
  "term_label": "endoplasmic reticulum membrane"
}